{
  "gene": "UniProtKB:P58876",
  "gene_name": "Histone H2B type 1-D",
  "term_id": "GO:0019731",
  "gene_symbol": "H2BC5",
  "term_label": "antibacterial humoral response"
}